{
  "gene": "UniProtKB:P23560",
  "gene_name": "Brain-derived neurotrophic factor",
  "term_id": "GO:0008083",
  "term_label": "growth factor activity",
  "gene_symbol": "BDNF"
}